inhibin secretion [GO:0032334] (biological process) Relationships: is a type of endocrine hormone secretion [GO:0060986] Regulation: regulated by regulation of inhibin secretion [GO:0032338]; negatively regulated by negative regulation of inhibin secretion [GO:0032339]; RO_0002213 by positive regulation of inhibin secretion [GO:0032340] Sources: GOC:mah Definition: The regulated release of an inhibin, either of two glycoproteins (designated A and B), secreted by the gonads and present in seminal plasma and follicular fluid, that inhibit pituitary production of follicle-stimulating hormone.